{
  "term_id": "UNKNOWN:0001",
  "gene_symbol": "IGLV1-47",
  "gene": "UniProtKB:P01700",
  "gene_name": "Immunoglobulin lambda variable 1-47",
  "term_label": "Unknown molecular function"
}